{
  "gene_symbol": "TMA7",
  "gene_name": "Translation machinery-associated protein 7",
  "gene": "UniProtKB:Q9Y2S6",
  "term_id": "UNKNOWN:0002",
  "term_label": "Unknown biological process"
}